{
  "term_label": "regulation of transcription by RNA polymerase II",
  "gene_symbol": "ZNF226",
  "gene_name": "Zinc finger protein 226",
  "term_id": "GO:0006357",
  "gene": "UniProtKB:Q9NYT6"
}